regulation of karyogamy [GO:0032871] (biological process) Relationships: is a type of regulation of nucleus organization [GO:1903353]; RO_0002211 karyogamy [GO:0000741] Sources: GOC:mah Definition: Any process that modulates the frequency, rate or extent of karyogamy, the creation of a single nucleus from multiple nuclei as a result of membrane fusion.